{
  "gene_name": "Folate receptor alpha",
  "term_id": "GO:0007155",
  "term_label": "cell adhesion",
  "gene": "UniProtKB:P15328",
  "gene_symbol": "FOLR1"
}